{
  "term_label": "hydroxymethylbilane synthase activity",
  "gene": "UniProtKB:P08397",
  "term_id": "GO:0004418",
  "gene_name": "Porphobilinogen deaminase",
  "gene_symbol": "HMBS"
}